{
  "term_label": "positive regulation of transcription by RNA polymerase II",
  "term_id": "GO:0045944",
  "gene_symbol": "ATOH1",
  "gene": "UniProtKB:Q92858",
  "gene_name": "Transcription factor ATOH1"
}